{
  "term_label": "sulfotransferase activity",
  "gene_symbol": "SULT4A1",
  "gene": "UniProtKB:Q9BR01",
  "term_id": "GO:0008146",
  "gene_name": "Sulfotransferase 4A1"
}